{
  "gene_symbol": "PSMA1",
  "term_label": "nucleus",
  "term_id": "GO:0005634",
  "gene_name": "Proteasome subunit alpha type-1",
  "gene": "UniProtKB:P25786"
}